{
  "term_label": "Unknown biological process",
  "gene_name": "Transmembrane protein 210",
  "gene": "UniProtKB:A6NLX4",
  "gene_symbol": "TMEM210",
  "term_id": "UNKNOWN:0002"
}